leucoanthocyanidin reductase activity [GO:0033788] (molecular function) Sources: EC:1.17.1.3 Also known as: (2R,3S)-catechin:NADP+ 4-oxidoreductase activity, leucocyanidin reductase activity Definition: Catalysis of the reaction: (2R,3S)-catechin + NADP+ + H2O = 2,3-trans-3,4-cis-leucocyanidin + NADPH + H+. Relationships: is a type of oxidoreductase activity, acting on CH or CH2 groups, NAD or NADP as acceptor [GO:0016726]